positive regulation of cardiac vascular smooth muscle cell differentiation [GO:2000724] (biological process) Sources: GOC:BHF Definition: Any process that activates or increases the frequency, rate or extent of cardiac vascular smooth muscle cell differentiation. Also known as: positive regulation of heart vascular smooth muscle cell differentiation Relationships: is a type of positive regulation of vascular associated smooth muscle cell differentiation [GO:1905065]; is a type of positive regulation of cardiocyte differentiation [GO:1905209]; is a type of regulation of cardiac vascular smooth muscle cell differentiation [GO:2000722]; RO_0002213 GO:0060947